{
  "term_label": "mitotic chromosome condensation",
  "term_id": "GO:0007076",
  "gene_name": "Structural maintenance of chromosomes protein 2",
  "gene": "UniProtKB:O95347",
  "gene_symbol": "SMC2"
}